{
  "term_label": "basement membrane",
  "term_id": "GO:0005604",
  "gene": "UniProtKB:Q5TAT6",
  "gene_name": "Collagen alpha-1(XIII) chain",
  "gene_symbol": "COL13A1"
}